{
  "gene_name": "Dynein axonemal intermediate chain 1",
  "term_label": "dynein light chain binding",
  "term_id": "GO:0045503",
  "gene": "UniProtKB:Q9UI46",
  "gene_symbol": "DNAI1"
}